protein secretion by the type IV secretion system [GO:0030255] (biological process) Definition: The process in which proteins are transferred into the extracellular milieu or directly into host cells, via the type IV protein secretion system. Also known as: protein secretion by the T4SS, protein secretion by the type IV protein secretion system, type IV protein secretion system Relationships: is_a protein secretion [GO:0009306]; is a type of secretion by the type IV secretion system [GO:0044097]; is a type of GO:0071806 Sources: GOC:pamgo_curators Note: Note that this term represents an activity and not a cellular structure. Consider also annotating to the cellular component term 'type IV protein secretion system complex ; GO:0043684'.